{
  "term_label": "Unknown biological process",
  "gene": "UniProtKB:Q495Y7",
  "gene_symbol": "SPDYE7P",
  "term_id": "UNKNOWN:0002",
  "gene_name": "Putative speedy protein E7"
}